MHC class Ib protein complex assembly [GO:0002398] (biological process) References: PMID:15928678, PMID:15928680 Sources: GOC:add Relationships: is a type of MHC protein complex assembly [GO:0002396] Definition: The aggregation, arrangement and bonding together of a set of components to form an MHC class Ib protein complex. Class Ib here refers to non-classical class I molecules.